{
  "gene_symbol": "TRIM77",
  "gene": "UniProtKB:I1YAP6",
  "term_id": "GO:0061630",
  "term_label": "ubiquitin protein ligase activity",
  "gene_name": "Tripartite motif-containing protein 77"
}